regulation of endoplasmic reticulum stress-induced eIF2 alpha phosphorylation [GO:0060734] (biological process) Sources: GOC:dph, GOC:tb Also known as: regulation of ER stress-induced eIF2 alpha phosphorylation, regulation of eIF2 alpha phosphorylation by ER stress, regulation of eIF2 alpha phosphorylation by endoplasmic reticulum stress Relationships: is a type of GO:0001932; is a type of GO:0006446; is a type of regulation of response to endoplasmic reticulum stress [GO:1905897]; regulates GO:0036492 Definition: Any process that modulates the rate, frequency, or extent of eIF2 alpha phosphorylation as a cellular response to endoplasmic reticulum stress.